{
  "term_id": "UNKNOWN:0003",
  "gene_name": "Probable RNA polymerase II nuclear localization protein SLC7A6OS",
  "term_label": "Unknown cellular component",
  "gene_symbol": "SLC7A6OS",
  "gene": "UniProtKB:Q96CW6"
}